{
  "gene_name": "RB1-inducible coiled-coil protein 1",
  "term_id": "GO:0000045",
  "gene_symbol": "RB1CC1",
  "gene": "UniProtKB:Q8TDY2",
  "term_label": "autophagosome assembly"
}